{
  "gene_symbol": "TAF11",
  "gene_name": "Transcription initiation factor TFIID subunit 11",
  "term_id": "GO:0051123",
  "term_label": "RNA polymerase II preinitiation complex assembly",
  "gene": "UniProtKB:Q15544"
}